{
  "gene_symbol": "SPATA31E1",
  "term_label": "Unknown molecular function",
  "term_id": "UNKNOWN:0001",
  "gene": "UniProtKB:Q6ZUB1",
  "gene_name": "Spermatogenesis-associated protein 31E1"
}